regulation of mast cell activation involved in immune response [GO:0033006] (biological process) Sources: GOC:mah Also known as: regulation of mast cell activation during immune response Relationships: is a type of positive regulation of immune effector process [GO:0002699]; is a type of regulation of mast cell activation [GO:0033003]; is a type of GO:0050776; RO_0002211 mast cell activation involved in immune response [GO:0002279] Subtypes: negative regulation of mast cell activation involved in immune response [GO:0033007], GO:0033008 Definition: Any process that modulates the frequency, rate, or extent of mast cell activation as part of an immune response.